{
  "term_label": "protein ubiquitination",
  "gene_symbol": "DTX1",
  "gene": "UniProtKB:Q86Y01",
  "gene_name": "E3 ubiquitin-protein ligase DTX1",
  "term_id": "GO:0016567"
}